{
  "gene_symbol": "LMBR1L",
  "gene_name": "Protein LMBR1L",
  "term_label": "transmembrane signaling receptor activity",
  "gene": "UniProtKB:Q6UX01",
  "term_id": "GO:0004888"
}